{
  "gene_symbol": "CCN3",
  "term_id": "GO:0008201",
  "gene_name": "CCN family member 3",
  "term_label": "heparin binding",
  "gene": "UniProtKB:P48745"
}